{
  "term_id": "GO:0070888",
  "gene_symbol": "ATOH8",
  "gene": "UniProtKB:Q96SQ7",
  "term_label": "E-box binding",
  "gene_name": "Transcription factor ATOH8"
}